primary ovarian follicle growth involved in primary follicle stage [GO:0043930] (BP) Also known as: primary ovarian follicle growth during primary follicle stage Definition: Increase in size of primary follicles including oocyte growth and granulosa and/or theca cell proliferation until more than one layer of granulosa cells is present (preantral follicle) as part of the primary follicle stage of oogenesis. Sources: GOC:mtg_mpo Relationships: is a type of primary ovarian follicle growth [GO:0001545]; is part of primary follicle stage [GO:0048160]